{
  "gene": "UniProtKB:Q6P3X8",
  "gene_name": "PiggyBac transposable element-derived protein 2",
  "term_label": "Unknown cellular component",
  "gene_symbol": "PGBD2",
  "term_id": "UNKNOWN:0003"
}